{
  "gene_name": "Short-wave-sensitive opsin 1",
  "gene_symbol": "OPN1SW",
  "term_label": "absorption of visible light",
  "gene": "UniProtKB:P03999",
  "term_id": "GO:0016038"
}